regulation of protein localization to prospore membrane [GO:2001231] (biological process) Subtypes: positive regulation of protein localization to prospore membrane [GO:2001232] Relationships: is a type of GO:1903076; regulates protein localization to prospore membrane [GO:1902657] Definition: Any process that modulates the frequency, rate or extent of protein localization to prospore membrane. Sources: GOC:mah Also known as: regulation of protein localisation to prospore membrane, regulation of protein targeting to FSM, regulation of protein targeting to ascospore-type prospore membrane, regulation of protein targeting to forespore membrane, regulation of protein targeting to prospore membrane, regulation of protein-prospore membrane targeting